Labd-13(16),14-diene-9-ol synthase activity [GO:0062202] (molecular function) Definition: Catalysis of the reaction: peregrinol diphosphate = diphosphate + labd-13(16),14-diene-9-ol. Relationships: is a type of carbon-oxygen lyase activity, acting on phosphates [GO:0016838] References: PMID:29315936 Sources: RHEA:62184